{
  "gene_name": "X-box-binding protein 1",
  "gene": "UniProtKB:P17861",
  "term_label": "nucleus",
  "gene_symbol": "XBP1",
  "term_id": "GO:0005634"
}